histone H3K79 trimethyltransferase activity [GO:0140956] (molecular function) Definition: Catalysis of the reaction: L-lysyl79-[histone H3] + 3 S-adenosyl-L-methionine = 3 H+ + N6,N6,N6-trimethyl-L-lysyl79-[histone H3] + 3 S-adenosyl-L-homocysteine. This reaction is the successive addition of up to three methyl group to the lysine residue at position 79 of the histone H3 protein, producing H3K79me3. References: PMID:15371351 Sources: RHEA:60328 Also known as: histone H3-K79 trimethylation, histone H3K79 trimethylation, histone H3K79 trimethylase activity, histone lysine N-trimethyltransferase activity (H3-K79 specific), histone trimethylase activity (H3-K79 specific), histone trimethyltransferase activity (H3-K79 specific), histone-H3K79 trimethyltransferase activity Note: Comment: Note that the residue position corresponds to the canonical human H3 histone (UniProtKB:P84243); this residue is conserved across all eukaryotes. Residue 1 is the first residue following removal of the initiating Methionine (Met). Note that each histone is encoded by multiple genes, and sequences may vary across different genes within an organism. Relationships: is a type of histone H3K79 methyltransferase activity [GO:0031151]